attachment of meiotic spindle microtubules to meiosis II kinetochore [GO:0051456] (biological process) Definition: The cellular process in which spindle microtubules become physically associated with the proteins making up the kinetochore complex in meiosis II. During meiosis II sister kinetochores are situated facing opposite spindle poles and bipolar attachment of the sister chromosomes to the spindle occurs. Sources: GOC:ai, GOC:clt, GOC:dph, GOC:tb Also known as: attachment of meiotic spindle microtubules to kinetochore in meiosis II, attachment of spindle microtubules to kinetochore during meiosis II, meiotic bipolar attachment Relationships: is a type of attachment of meiotic spindle microtubules to kinetochore [GO:0051316]; is part of meiotic metaphase II chromosome alignment [GO:0043061]